{
  "gene_name": "Striatin-interacting protein 1",
  "gene_symbol": "STRIP1",
  "gene": "UniProtKB:Q5VSL9",
  "term_id": "GO:0035331",
  "term_label": "negative regulation of hippo signaling"
}